{
  "gene_name": "Tyrosyl-DNA phosphodiesterase 1",
  "gene_symbol": "TDP1",
  "term_label": "nucleus",
  "term_id": "GO:0005634",
  "gene": "UniProtKB:Q9NUW8"
}